{
  "gene_name": "Trafficking protein particle complex subunit 6A",
  "gene_symbol": "TRAPPC6A",
  "gene": "UniProtKB:O75865",
  "term_label": "trans-Golgi network",
  "term_id": "GO:0005802"
}